{
  "term_id": "GO:0005549",
  "gene_name": "Olfactory receptor 5H6",
  "gene": "UniProtKB:Q8NGV6",
  "term_label": "odorant binding",
  "gene_symbol": "OR5H6"
}